{
  "gene_symbol": "MARCO",
  "term_label": "Unknown molecular function",
  "gene_name": "Macrophage receptor MARCO",
  "term_id": "UNKNOWN:0001",
  "gene": "UniProtKB:Q9UEW3"
}